{
  "term_id": "GO:0008083",
  "gene": "UniProtKB:P49767",
  "term_label": "growth factor activity",
  "gene_name": "Vascular endothelial growth factor C",
  "gene_symbol": "VEGFC"
}